{
  "term_label": "structural constituent of nuclear pore",
  "gene_name": "Nuclear pore complex protein Nup205",
  "term_id": "GO:0017056",
  "gene": "UniProtKB:Q92621",
  "gene_symbol": "NUP205"
}